{
  "term_label": "nucleus",
  "gene": "UniProtKB:Q29RF7",
  "gene_name": "Sister chromatid cohesion protein PDS5 homolog A",
  "term_id": "GO:0005634",
  "gene_symbol": "PDS5A"
}